{
  "term_label": "nucleus",
  "gene": "UniProtKB:Q9NP71",
  "term_id": "GO:0005634",
  "gene_name": "Carbohydrate-responsive element-binding protein",
  "gene_symbol": "MLXIPL"
}